negative regulation of type IIb hypersensitivity [GO:0001800] (biological process) Also known as: down regulation of type IIb hypersensitivity, down-regulation of type IIb hypersensitivity, downregulation of type IIb hypersensitivity, inhibition of type IIb hypersensitivity Sources: GOC:add, ISBN:0781735149 Relationships: is a type of regulation of type IIb hypersensitivity [GO:0001799]; is a type of negative regulation of type II hypersensitivity [GO:0002893]; negatively regulates GO:0001795 Definition: Any process that stops, prevents, or reduces the rate of type IIb hypersensitivity, a type of inflammatory response.